{
  "gene": "UniProtKB:P28325",
  "gene_name": "Cystatin-D",
  "gene_symbol": "CST5",
  "term_label": "vesicle",
  "term_id": "GO:0031982"
}